{
  "term_id": "UNKNOWN:0002",
  "term_label": "Unknown biological process",
  "gene_symbol": "CCDC198",
  "gene_name": "Uncharacterized protein CCDC198",
  "gene": "UniProtKB:Q9NVL8"
}